{
  "gene_symbol": "ZNHIT6",
  "gene_name": "Box C_D snoRNA protein 1",
  "term_label": "box C/D snoRNP assembly",
  "term_id": "GO:0000492",
  "gene": "UniProtKB:Q9NWK9"
}